{
  "term_id": "GO:0006357",
  "gene_name": "Zinc finger and BTB domain-containing protein 47",
  "gene": "UniProtKB:Q9UFB7",
  "gene_symbol": "ZBTB47",
  "term_label": "regulation of transcription by RNA polymerase II"
}